{
  "term_label": "endoplasmic reticulum to Golgi vesicle-mediated transport",
  "gene_name": "BET1 homolog",
  "gene": "UniProtKB:O15155",
  "term_id": "GO:0006888",
  "gene_symbol": "BET1"
}